{
  "gene": "UniProtKB:Q6ZVK1",
  "term_id": "UNKNOWN:0001",
  "term_label": "Unknown molecular function",
  "gene_symbol": "TMEM179",
  "gene_name": "Transmembrane protein 179"
}